{
  "term_label": "protein insertion into membrane",
  "term_id": "GO:0051205",
  "gene": "UniProtKB:Q14D33",
  "gene_symbol": "RTP5",
  "gene_name": "Receptor-transporting protein 5"
}